{
  "gene": "UniProtKB:Q5HYM0",
  "gene_symbol": "ZC3H12B",
  "term_label": "cytoplasmic ribonucleoprotein granule",
  "gene_name": "Probable ribonuclease ZC3H12B",
  "term_id": "GO:0036464"
}